{
  "gene_symbol": "ZNF320",
  "term_id": "GO:0000978",
  "term_label": "RNA polymerase II cis-regulatory region sequence-specific DNA binding",
  "gene_name": "Zinc finger protein 320",
  "gene": "UniProtKB:A2RRD8"
}